regulation of cytokinin-activated signaling pathway [GO:0080036] (biological process) Subtypes: negative regulation of cytokinin-activated signaling pathway [GO:0080037], positive regulation of cytokinin-activated signaling pathway [GO:0080038] Definition: Any process that modulates the frequency, rate or extent of cytokinin signaling. Relationships: is_a regulation of signal transduction [GO:0009966]; regulates cytokinin-activated signaling pathway [GO:0009736] Sources: GOC:dhl Also known as: regulation of cytokinin mediated signalling, regulation of cytokinin mediated signaling pathway